{
  "term_label": "positive regulation of cell migration",
  "term_id": "GO:0030335",
  "gene": "UniProtKB:P35968",
  "gene_name": "Vascular endothelial growth factor receptor 2",
  "gene_symbol": "KDR"
}